carbon phosphorus lyase activity [GO:0018835] (molecular function) References: PMID:3804975 Subtypes: alpha-D-ribose 1-methylphosphonate 5-phosphate C-P-lyase activity [GO:0098848] Definition: Catalysis of the reaction: alkylphosphonic acid = R-CH3 + phosphate. Substrates include aminomethylphosphonic acid (AMPA) (forms methylamine), dimethylphosphinic acid (forms methylphosphonic acid), glyphosate (forms sarcosine) and methylphosphonic acid (forms phosphate). Relationships: is a type of lyase activity [GO:0016829]